negative regulation of cell division [GO:0051782] (biological process) Definition: Any process that stops, prevents, or reduces the frequency, rate or extent of cell division. Sources: GOC:ai Also known as: down regulation of cell division, down-regulation of cell division, downregulation of cell division, inhibition of cell division Relationships: is a type of negative regulation of cellular process [GO:0048523]; is a type of regulation of cell division [GO:0051302]; negatively regulates cell division [GO:0051301] Subtypes: negative regulation of cytokinesis [GO:0032466], negative regulation of asymmetric cell division [GO:0045769], GO:0045781, negative regulation of somatic stem cell division [GO:1904676]